cerebellum formation [GO:0021588] (biological process) Relationships: is a type of anatomical structure formation involved in morphogenesis [GO:0048646]; is part of hindbrain formation [GO:0021576]; is part of GO:0021587 Definition: The process that gives rise to the cerebellum. This process pertains to the initial formation of a structure from unspecified parts. The cerebellum is the portion of the brain in the back of the head between the cerebrum and the pons. The cerebellum controls balance for walking and standing, modulates the force and range of movement and is involved in the learning of motor skills. Sources: GOC:cls, GOC:dgh, GOC:dph, GOC:jid, GO_REF:0000021